regulation of microtubule depolymerization [GO:0031114] (biological process) Sources: GOC:mah Definition: Any process that modulates the frequency, rate or extent of microtubule depolymerization. Subtypes: GO:0007026, regulation of cytoplasmic microtubule depolymerization [GO:0010937], GO:0031117 Also known as: regulation of microtubule disassembly Relationships: is a type of regulation of microtubule polymerization or depolymerization [GO:0031110]; is a type of regulation of protein depolymerization [GO:1901879]; is a type of regulation of supramolecular fiber organization [GO:1902903]; regulates microtubule depolymerization [GO:0007019]